{
  "gene_name": "E3 ubiquitin-protein ligase TRIM34",
  "term_id": "GO:0005737",
  "term_label": "cytoplasm",
  "gene": "UniProtKB:Q9BYJ4",
  "gene_symbol": "TRIM34"
}